tRNA aminoacylation for protein translation [GO:0006418] (biological process) Subtypes: GO:0006419, arginyl-tRNA aminoacylation [GO:0006420], GO:0006421, aspartyl-tRNA aminoacylation [GO:0006422], cysteinyl-tRNA aminoacylation [GO:0006423], glutamyl-tRNA aminoacylation [GO:0006424], glutaminyl-tRNA aminoacylation [GO:0006425], glycyl-tRNA aminoacylation [GO:0006426], histidyl-tRNA aminoacylation [GO:0006427], isoleucyl-tRNA aminoacylation [GO:0006428], leucyl-tRNA aminoacylation [GO:0006429], lysyl-tRNA aminoacylation [GO:0006430], methionyl-tRNA aminoacylation [GO:0006431], phenylalanyl-tRNA aminoacylation [GO:0006432], prolyl-tRNA aminoacylation [GO:0006433], seryl-tRNA aminoacylation [GO:0006434], threonyl-tRNA aminoacylation [GO:0006435], GO:0006436, tyrosyl-tRNA aminoacylation [GO:0006437], valyl-tRNA aminoacylation [GO:0006438], tRNA aminoacylation for mitochondrial protein translation [GO:0070127] Sources: GOC:ma Also known as: tRNA charging Relationships: is a type of tRNA aminoacylation [GO:0043039]; is part of translation [GO:0006412] Definition: The synthesis of aminoacyl tRNA by the formation of an ester bond between the 3'-hydroxyl group of the most 3' adenosine of the tRNA and the alpha carboxylic acid group of an amino acid, to be used in ribosome-mediated polypeptide synthesis.